{
  "gene": "UniProtKB:Q15653",
  "gene_name": "NF-kappa-B inhibitor beta",
  "gene_symbol": "NFKBIB",
  "term_id": "UNKNOWN:0003",
  "term_label": "Unknown cellular component"
}